{
  "gene_symbol": "INKA2",
  "gene_name": "PAK4-inhibitor INKA2",
  "term_id": "GO:0005634",
  "term_label": "nucleus",
  "gene": "UniProtKB:Q9NTI7"
}